lens fiber cell morphogenesis [GO:0070309] (biological process) Definition: The process in which the structures of a lens fiber cell are generated and organized. This process occurs while the initially relatively unspecialized cell is acquiring the specialized features of a lens fiber cell. A lens fiber cell is any of the elongated, tightly packed cells that make up the bulk of the mature lens in a camera-type eye. Relationships: is a type of GO:0000902; is part of lens morphogenesis in camera-type eye [GO:0002089]; is part of lens fiber cell development [GO:0070307] Also known as: lens fiber cell morphogenesis during differentiation, lens fibre cell morphogenesis, elongation of lens fiber cell References: PMID:7693735 Sources: GOC:mah